{
  "term_id": "GO:0043066",
  "gene": "UniProtKB:Q8TEB9",
  "gene_symbol": "RHBDD1",
  "term_label": "negative regulation of apoptotic process",
  "gene_name": "Rhomboid-related protein 4"
}